positive regulation of blood-brain barrier permeability [GO:1905605] (biological process) Relationships: is a type of positive regulation of vascular permeability [GO:0043117]; is a type of regulation of blood-brain barrier permeability [GO:1905603] References: PMID:22524708, PMID:30280653 Sources: GOC:TermGenie, GOC:als, GOC:aruk, GOC:bc, GO_REF:0000058 Definition: Any process that increases blood-brain barrier permeability, the quality of the blood-brain barrier that allows for a controlled passage of substances (e.g. macromolecules, small molecules, ions) into and out of the brain. Also known as: positive regulation of BBB permeability, positive regulation of blood/brain barrier permeability, up-regulation of BBB permeability, up-regulation of blood-brain barrier permeability, up-regulation of blood/brain barrier permeability, upregulation of BBB permeability, upregulation of blood-brain barrier permeability, upregulation of blood/brain barrier permeability, activation of maintenance of permeability of BBB, activation of maintenance of permeability of blood-brain barrier